{
  "gene_symbol": "RYK",
  "gene_name": "Tyrosine-protein kinase RYK",
  "term_id": "GO:0051897",
  "term_label": "positive regulation of phosphatidylinositol 3-kinase/protein kinase B signal transduction",
  "gene": "UniProtKB:P34925"
}